negative regulation of protein localization to cell cortex of cell tip [GO:0106013] (biological process) Relationships: is a type of regulation of protein localization to cell cortex of cell tip [GO:1990895] References: PMID:19474792 Sources: GOC:vw Definition: Any process that stops, prevents or reduces the frequency, rate or extent of protein localization to the cell cortex of the cell tip.